cellular response to tropane [GO:0071416] (biological process) Definition: Any process that results in a change in state or activity of a cell (in terms of movement, secretion, enzyme production, gene expression, etc.) as a result of a tropane stimulus. Tropane is a nitrogenous bicyclic organic compound mainly known for a group of alkaloids derived from it (called tropane alkaloids), which include, among others, atropine and cocaine. Sources: GOC:mah Relationships: is a type of response to tropane [GO:0014073]; is a type of cellular response to alkaloid [GO:0071312]